{
  "term_id": "GO:0005737",
  "gene_name": "Regulator of nonsense transcripts 3A",
  "gene": "UniProtKB:Q9H1J1",
  "gene_symbol": "UPF3A",
  "term_label": "cytoplasm"
}